{
  "gene_symbol": "CCR6",
  "term_label": "external side of plasma membrane",
  "term_id": "GO:0009897",
  "gene": "UniProtKB:P51684",
  "gene_name": "C-C chemokine receptor type 6"
}